{
  "gene_name": "Ribosome biogenesis protein NSA2 homolog",
  "gene_symbol": "NSA2",
  "term_label": "nucleolus",
  "term_id": "GO:0005730",
  "gene": "UniProtKB:O95478"
}